{
  "gene_name": "Inhibitor of growth protein 4",
  "term_label": "Unknown molecular function",
  "gene": "UniProtKB:Q9UNL4",
  "gene_symbol": "ING4",
  "term_id": "UNKNOWN:0001"
}